{
  "term_id": "UNKNOWN:0003",
  "gene": "UniProtKB:A2RRH5",
  "term_label": "Unknown cellular component",
  "gene_symbol": "WDR27",
  "gene_name": "WD repeat-containing protein 27"
}